{
  "term_id": "GO:0044548",
  "term_label": "S100 protein binding",
  "gene_symbol": "S100B",
  "gene": "UniProtKB:P04271",
  "gene_name": "Protein S100-B"
}